{
  "term_id": "GO:0098609",
  "gene": "UniProtKB:Q96J84",
  "term_label": "cell-cell adhesion",
  "gene_symbol": "KIRREL1",
  "gene_name": "Kin of IRRE-like protein 1"
}